{
  "gene_symbol": "MYO5B",
  "gene_name": "Unconventional myosin-Vb",
  "term_label": "membrane",
  "term_id": "GO:0016020",
  "gene": "UniProtKB:Q9ULV0"
}